{
  "term_label": "actin filament organization",
  "gene_symbol": "ARHGAP25",
  "gene_name": "Rho GTPase-activating protein 25",
  "term_id": "GO:0007015",
  "gene": "UniProtKB:P42331"
}